{
  "gene_name": "DDB1- and CUL4-associated factor 16",
  "gene_symbol": "DCAF16",
  "gene": "UniProtKB:Q9NXF7",
  "term_id": "UNKNOWN:0002",
  "term_label": "Unknown biological process"
}